{
  "gene_symbol": "ADAM15",
  "gene": "UniProtKB:Q13444",
  "term_label": "integrin binding",
  "gene_name": "Disintegrin and metalloproteinase domain-containing protein 15",
  "term_id": "GO:0005178"
}